{
  "gene": "UniProtKB:Q13643",
  "gene_symbol": "FHL3",
  "term_label": "actin binding",
  "gene_name": "Four and a half LIM domains protein 3",
  "term_id": "GO:0003779"
}